{
  "gene_symbol": "PHF13",
  "gene": "UniProtKB:Q86YI8",
  "gene_name": "PHD finger protein 13",
  "term_label": "nucleus",
  "term_id": "GO:0005634"
}